{
  "term_id": "GO:0006357",
  "term_label": "regulation of transcription by RNA polymerase II",
  "gene_name": "Homeobox protein Nkx-6.3",
  "gene_symbol": "NKX6-3",
  "gene": "UniProtKB:A6NJ46"
}